2-chloro-N-isopropylacetanilide catabolic process [GO:0046302] (biological process) Also known as: 2-chloro-N-isopropylacetanilide breakdown, 2-chloro-N-isopropylacetanilide catabolism, 2-chloro-N-isopropylacetanilide degradation Relationships: is a type of catabolic process [GO:0009056]; is a type of benzene-containing compound metabolic process [GO:0042537]; is a type of GO:0043603; is a type of organohalogen metabolic process [GO:0090345] Definition: The chemical reactions and pathways resulting in the breakdown of 2-chloro-N-isopropylacetanilide, an acylanide herbicide widely used to protect corn, onion, cabbage, rose bushes, and ornamental plants. Sources: GOC:ai